response to mitotic cell cycle spindle orientation checkpoint signaling [GO:0072482] (biological process) Relationships: is a type of response to mitotic spindle checkpoint signaling [GO:0072476] Definition: A process that occurs in response to signals generated as a result of mitotic cell cycle spindle orientation checkpoint signaling. Also known as: mitotic cell cycle spindle orientation checkpoint effector process, response to signal involved in mitotic cell cycle spindle orientation checkpoint Sources: GOC:mtg_cell_cycle